{
  "term_id": "UNKNOWN:0002",
  "gene": "UniProtKB:Q9Y5V0",
  "term_label": "Unknown biological process",
  "gene_symbol": "ZNF706",
  "gene_name": "Zinc finger protein 706"
}